histone mRNA metabolic process [GO:0008334] (biological process) Also known as: histone mRNA metabolism, stem-loop-containing histone mRNA 3'-end processing Note: In higher Eukaryotes, histone mRNAs (stem-loop containing) are non-polyadenylated and thus have a different form of 3'-end regulation to other mRNAs. In lower Eukaryotes, the 3'-ends of histone mRNAs are polyadenylated. References: PMID:17855393 Sources: GOC:krc, GOC:mah Subtypes: GO:0006398, histone mRNA catabolic process [GO:0071044] Definition: The chemical reactions and pathways involving an mRNA encoding a histone. Relationships: is a type of mRNA metabolic process [GO:0016071]